{
  "gene_name": "Kelch repeat and BTB domain-containing protein 12",
  "gene": "UniProtKB:Q3ZCT8",
  "term_label": "Cul3-RING ubiquitin ligase complex",
  "term_id": "GO:0031463",
  "gene_symbol": "KBTBD12"
}